{
  "gene_symbol": "SLC23A3",
  "term_id": "UNKNOWN:0001",
  "term_label": "Unknown molecular function",
  "gene": "UniProtKB:Q6PIS1",
  "gene_name": "Solute carrier family 23 member 3"
}